{
  "term_label": "transcription cis-regulatory region binding",
  "term_id": "GO:0000976",
  "gene_name": "Zinc finger protein 606",
  "gene_symbol": "ZNF606",
  "gene": "UniProtKB:Q8WXB4"
}